{
  "term_label": "cytoplasm",
  "term_id": "GO:0005737",
  "gene_symbol": "AGAP3",
  "gene": "UniProtKB:Q96P47",
  "gene_name": "Arf-GAP with GTPase, ANK repeat and PH domain-containing protein 3"
}